drinking behavior [GO:0042756] (biological process) Sources: GOC:curators, GOC:pr Subtypes: GO:0003051 Also known as: drinking behaviour Relationships: is a type of feeding behavior [GO:0007631] Definition: The specific behavior of an organism relating to the intake of liquids, especially water.